{
  "term_id": "UNKNOWN:0001",
  "gene_symbol": "NPNT",
  "gene_name": "Nephronectin",
  "gene": "UniProtKB:Q6UXI9",
  "term_label": "Unknown molecular function"
}